{
  "term_id": "GO:0000932",
  "gene_symbol": "DCP1B",
  "gene_name": "mRNA-decapping enzyme 1B",
  "gene": "UniProtKB:Q8IZD4",
  "term_label": "P-body"
}